{
  "gene_name": "Serine_threonine-protein kinase PAK 3",
  "term_id": "GO:0050770",
  "term_label": "regulation of axonogenesis",
  "gene_symbol": "PAK3",
  "gene": "UniProtKB:O75914"
}